{
  "term_label": "Unknown cellular component",
  "gene_name": "Ribonuclease H1",
  "gene": "UniProtKB:O60930",
  "term_id": "UNKNOWN:0003",
  "gene_symbol": "RNASEH1"
}